{
  "gene": "UniProtKB:Q96CS4",
  "gene_symbol": "ZNF689",
  "term_id": "GO:0000978",
  "gene_name": "Zinc finger protein 689",
  "term_label": "RNA polymerase II cis-regulatory region sequence-specific DNA binding"
}